cardiac muscle cell-cardiac muscle cell adhesion [GO:0086042] (biological process) Subtypes: SA node cell-atrial cardiac muscle cell adhesion involved in cell communication [GO:0086022], atrial cardiac muscle cell-AV node cell adhesion involved in cell communication [GO:0086071], AV node cell-bundle of His cell adhesion involved in cell communication [GO:0086072], GO:0086073, Purkinje myocyte-ventricular cardiac muscle cell adhesion involved in cell communication [GO:0086074] Definition: The attachment of one cardiomyocyte to another cardiomyocyte via adhesion molecules. Sources: GOC:BHF, GOC:mtg_cardiac_conduct_nov11 Also known as: cardiomyocyte-cardiomyocyte adhesion Relationships: is a type of homotypic cell-cell adhesion [GO:0034109]